{
  "term_id": "GO:1902531",
  "term_label": "regulation of intracellular signal transduction",
  "gene_symbol": "TNFAIP8L3",
  "gene": "UniProtKB:Q5GJ75",
  "gene_name": "Tumor necrosis factor alpha-induced protein 8-like protein 3"
}